inosinate nucleosidase activity [GO:0047723] (molecular function) Definition: Catalysis of the reaction: H2O + IMP = D-ribose 5-phosphate + hypoxanthine. Sources: EC:3.2.2.12, RHEA:20469 Also known as: 5'-inosinate phosphoribohydrolase activity Relationships: is a type of hydrolase activity, hydrolyzing N-glycosyl compounds [GO:0016799]